{
  "term_id": "UNKNOWN:0002",
  "gene_name": "Spermatogenesis-associated protein 8",
  "gene": "UniProtKB:Q6RVD6",
  "term_label": "Unknown biological process",
  "gene_symbol": "SPATA8"
}